{
  "gene": "UniProtKB:P19440",
  "gene_name": "Glutathione hydrolase 1 proenzyme",
  "term_label": "glutathione hydrolase activity",
  "gene_symbol": "GGT1",
  "term_id": "GO:0036374"
}